{
  "gene_symbol": "SIX6OS1",
  "term_label": "spermatogenesis",
  "gene": "UniProtKB:Q8N1H7",
  "term_id": "GO:0007283",
  "gene_name": "Protein SIX6OS1"
}